{
  "term_id": "UNKNOWN:0003",
  "gene": "UniProtKB:A0A1B0GVD1",
  "gene_name": "Protein FAM237B",
  "term_label": "Unknown cellular component",
  "gene_symbol": "FAM237B"
}